{
  "term_id": "GO:0006606",
  "gene_name": "Nuclear envelope pore membrane protein POM 121",
  "term_label": "protein import into nucleus",
  "gene_symbol": "POM121",
  "gene": "UniProtKB:Q96HA1"
}